pseurotin A biosynthetic process [GO:1900790] (biological process) Definition: The chemical reactions and pathways resulting in the formation of pseurotin A. Relationships: is a type of GO:0072339 Regulation: regulated by regulation of pseurotin A biosynthetic process [GO:1900849]; negatively regulated by negative regulation of pseurotin A biosynthetic process [GO:1900850]; positively regulated by positive regulation of pseurotin A biosynthetic process [GO:1900851] Sources: GOC:TermGenie, GOC:di Also known as: pseurotin A anabolism, pseurotin A biosynthesis, pseurotin A formation, pseurotin A synthesis, Pseurotin anabolism, Pseurotin biosynthesis, Pseurotin biosynthetic process, Pseurotin formation, Pseurotin synthesis